{
  "term_label": "regulation of transcription by RNA polymerase II",
  "term_id": "GO:0006357",
  "gene_name": "Homeobox protein DLX-4",
  "gene_symbol": "DLX4",
  "gene": "UniProtKB:Q92988"
}